{
  "term_id": "UNKNOWN:0003",
  "gene": "UniProtKB:A0A075B6Z5",
  "term_label": "Unknown cellular component",
  "gene_symbol": "TRAJ4",
  "gene_name": "T cell receptor alpha joining 4 (Fragment)"
}